left horn of sinus venosus development [GO:0061079] (BP) Definition: The progression of the left horn of the sinus venosus from its initial formation to the mature structure. Sources: GOC:dph Relationships: is a type of anatomical structure development [GO:0048856]; BFO_0000050 GO:0003235